{
  "term_id": "GO:0000278",
  "gene_symbol": "TUBGCP2",
  "gene_name": "Gamma-tubulin complex component 2",
  "term_label": "mitotic cell cycle",
  "gene": "UniProtKB:Q9BSJ2"
}